{
  "term_id": "GO:0019894",
  "term_label": "kinesin binding",
  "gene_symbol": "KLC1",
  "gene_name": "Kinesin light chain 1",
  "gene": "UniProtKB:Q07866"
}